fatty acid metabolic process [GO:0006631] (biological process) Also known as: fatty acid metabolism Regulation: regulated by GO:0019217; negatively regulated by negative regulation of fatty acid metabolic process [GO:0045922]; positively regulated by GO:0045923 Sources: ISBN:0198547684 Relationships: is_a lipid metabolic process [GO:0006629]; is a type of monocarboxylic acid metabolic process [GO:0032787] Subtypes: very long-chain fatty acid metabolic process [GO:0000038], long-chain fatty acid metabolic process [GO:0001676], fatty acid biosynthetic process [GO:0006633], fatty acid catabolic process [GO:0009062], lipoate metabolic process [GO:0009106], lipoxygenase pathway [GO:0019372], GO:0019395, unsaturated fatty acid metabolic process [GO:0033559], short-chain fatty acid metabolic process [GO:0046459], medium-chain fatty acid metabolic process [GO:0051791], methyl-branched fatty acid metabolic process [GO:0097089], poly(hydroxyalkanoate) biosynthetic process from fatty acid [GO:1902925], GO:1903964, methane biosynthetic process from 3-(methylthio)propionic acid [GO:2001132] Definition: The chemical reactions and pathways involving fatty acids, aliphatic monocarboxylic acids liberated from naturally occurring fats and oils by hydrolysis.